{
  "gene": "UniProtKB:Q86XR5",
  "gene_name": "Proline-rich membrane anchor 1",
  "gene_symbol": "PRIMA1",
  "term_id": "UNKNOWN:0003",
  "term_label": "Unknown cellular component"
}